{
  "term_id": "GO:0003735",
  "gene_symbol": "RPS13",
  "gene": "UniProtKB:P62277",
  "gene_name": "Small ribosomal subunit protein uS15",
  "term_label": "structural constituent of ribosome"
}